positive regulation of granzyme A production [GO:2000513] (biological process) Sources: GOC:obol Relationships: is a type of GO:0002702; is a type of regulation of granzyme A production [GO:2000511]; positively regulates GO:0035746 Definition: Any process that activates or increases the frequency, rate or extent of granzyme A production.